{
  "gene_symbol": "TESK1",
  "term_id": "GO:0005634",
  "term_label": "nucleus",
  "gene_name": "Dual specificity testis-specific protein kinase 1",
  "gene": "UniProtKB:Q15569"
}